{
  "gene_name": "FH1_FH2 domain-containing protein 1",
  "term_label": "actin filament binding",
  "gene_symbol": "FHOD1",
  "gene": "UniProtKB:Q9Y613",
  "term_id": "GO:0051015"
}